{
  "gene": "UniProtKB:P15863",
  "term_label": "embryo development ending in birth or egg hatching",
  "term_id": "GO:0009792",
  "gene_symbol": "PAX1",
  "gene_name": "Paired box protein Pax-1"
}